{
  "gene": "UniProtKB:P01588",
  "gene_name": "Erythropoietin",
  "term_id": "GO:0030218",
  "term_label": "erythrocyte differentiation",
  "gene_symbol": "EPO"
}